{
  "gene": "UniProtKB:Q9H4R4",
  "gene_name": "Putative nuclear receptor corepressor 1-like protein NCOR1P1",
  "gene_symbol": "NCOR1P1",
  "term_id": "UNKNOWN:0002",
  "term_label": "Unknown biological process"
}